acetoxybutynylbithiophene deacetylase activity [GO:0047373] (molecular function) Definition: Catalysis of the reaction: 5-(4-acetoxybut-1-ynyl)-2,2'-bithiophene + H2O = 5-(4-hydroxy-but-1-ynyl)-2,2'-bithiophene + acetate + H+. Relationships: is a type of GO:0019213; is a type of carboxylic ester hydrolase activity [GO:0052689] Also known as: 5-(4-acetoxy-1-butynyl)-2,2'-bithiophene:acetate esterase activity, 5-(4-acetoxybut-1-ynyl)-2,2'-bithiophene O-acetylhydrolase activity, acetoxybutynylbithiophene esterase activity Sources: EC:3.1.1.54, RHEA:11548